{
  "term_id": "GO:0000981",
  "gene": "UniProtKB:Q9Y543",
  "term_label": "DNA-binding transcription factor activity, RNA polymerase II-specific",
  "gene_symbol": "HES2",
  "gene_name": "Transcription factor HES-2"
}